{
  "gene_symbol": "GNAT2",
  "term_label": "photoreceptor inner segment",
  "term_id": "GO:0001917",
  "gene_name": "Guanine nucleotide-binding protein G(t) subunit alpha-2",
  "gene": "UniProtKB:P19087"
}